{
  "gene": "UniProtKB:Q9UBD0",
  "gene_symbol": "HSFX2",
  "term_id": "UNKNOWN:0002",
  "term_label": "Unknown biological process",
  "gene_name": "Heat shock transcription factor, X-linked"
}